Notch signaling pathway involved in camera-type eye photoreceptor fate commitment [GO:0060227] (BP) Relationships: is a type of Notch signaling pathway [GO:0007219]; is part of GO:0060220 Also known as: Notch signalling pathway involved in camera-type eye photoreceptor fate commitment Definition: The series of molecular signals initiated by binding of an extracellular ligand to a Notch receptor on the surface of the target cell that contributes to the commitment of a precursor cell to a eye photoreceptor fate. Sources: GOC:dph